{
  "term_label": "innate immune response in mucosa",
  "gene": "UniProtKB:Q16778",
  "gene_name": "Histone H2B type 2-E",
  "term_id": "GO:0002227",
  "gene_symbol": "H2BC21"
}